negative regulation of adaptive immune memory response [GO:1905675] (BP) Also known as: down regulation of adaptive immune memory response, down-regulation of adaptive immune memory response, downregulation of adaptive immune memory response, inhibition of adaptive immune memory response Relationships: is a type of negative regulation of adaptive immune response [GO:0002820]; is a type of GO:1905674; negatively regulates adaptive immune memory response [GO:0090716] Definition: Any process that stops, prevents or reduces the frequency, rate or extent of adaptive immune memory response. References: PMID:26831526 Sources: GOC:TermGenie, GO_REF:0000058